{
  "gene": "UniProtKB:P84095",
  "gene_name": "Rho-related GTP-binding protein RhoG",
  "term_id": "GO:0007163",
  "gene_symbol": "RHOG",
  "term_label": "establishment or maintenance of cell polarity"
}